{
  "gene": "UniProtKB:Q2NKX9",
  "term_label": "Unknown cellular component",
  "gene_symbol": "C2orf68",
  "gene_name": "UPF0561 protein C2orf68",
  "term_id": "UNKNOWN:0003"
}